{
  "term_label": "positive regulation of synapse assembly",
  "gene": "UniProtKB:Q8TF66",
  "gene_name": "Leucine-rich repeat-containing protein 15",
  "gene_symbol": "LRRC15",
  "term_id": "GO:0051965"
}